{
  "gene_name": "Putative uncharacterized SMG1-like protein",
  "term_id": "UNKNOWN:0003",
  "gene": "UniProtKB:Q6P435",
  "gene_symbol": "Q6P435",
  "term_label": "Unknown cellular component"
}